{
  "term_id": "GO:0045944",
  "gene_symbol": "SREBF2",
  "term_label": "positive regulation of transcription by RNA polymerase II",
  "gene_name": "Sterol regulatory element-binding protein 2",
  "gene": "UniProtKB:Q12772"
}